{
  "term_label": "Unknown biological process",
  "gene_name": "Oxysterol-binding protein 2",
  "term_id": "UNKNOWN:0002",
  "gene": "UniProtKB:Q969R2",
  "gene_symbol": "OSBP2"
}